{
  "gene": "UniProtKB:Q92966",
  "term_label": "bent DNA binding",
  "term_id": "GO:0003681",
  "gene_symbol": "SNAPC3",
  "gene_name": "snRNA-activating protein complex subunit 3"
}